{
  "gene_name": "Phospholipase D2",
  "term_id": "GO:0060627",
  "gene_symbol": "PLD2",
  "term_label": "regulation of vesicle-mediated transport",
  "gene": "UniProtKB:O14939"
}